{
  "gene_name": "Adhesion G-protein coupled receptor F2",
  "gene": "UniProtKB:Q8IZF7",
  "term_id": "UNKNOWN:0003",
  "term_label": "Unknown cellular component",
  "gene_symbol": "ADGRF2P"
}